oligodendrocyte cell migration from the subpallium to the cortex [GO:0021829] (biological process) Definition: The directed movement of oligodendrocytes from the subpallium to the cerebral cortex during forebrain development. References: PMID:12626695 Sources: GOC:cls, GOC:dgh, GOC:dph, GOC:jid, GO_REF:0000021 Relationships: is a type of GO:0021826; is_a telencephalon glial cell migration [GO:0022030]